glucose-6-phosphate isomerase activity [GO:0004347] (molecular function) Definition: Catalysis of the reaction: alpha-D-glucose 6-phosphate = beta-D-fructose 6-phosphate. Sources: RHEA:11816 Also known as: hexose monophosphate isomerase activity, hexosephosphate isomerase activity, phosphohexoisomerase activity, phosphohexomutase activity, phosphohexose isomerase activity, phosphosaccharomutase activity, D-glucose-6-phosphate aldose-ketose-isomerase activity, D-glucose-6-phosphate ketol-isomerase activity, glucose phosphate isomerase activity, hexose phosphate isomerase activity, oxoisomerase activity, phosphoglucoisomerase activity, phosphoglucose isomerase activity Relationships: is a type of intramolecular oxidoreductase activity, interconverting aldoses and ketoses [GO:0016861]